carbon dioxide receptor activity [GO:0170015] (molecular function) Relationships: is a type of signaling receptor activity [GO:0038023] Definition: Combining with carbon dioxide to initiate a change in cell activity. References: PMID:24240097